{
  "term_id": "GO:0006357",
  "gene": "UniProtKB:Q02556",
  "gene_symbol": "IRF8",
  "term_label": "regulation of transcription by RNA polymerase II",
  "gene_name": "Interferon regulatory factor 8"
}